{
  "gene_symbol": "NEIL2",
  "term_id": "UNKNOWN:0002",
  "gene": "UniProtKB:Q969S2",
  "term_label": "Unknown biological process",
  "gene_name": "Endonuclease 8-like 2"
}